endothelial cell fate commitment [GO:0060839] (biological process) Sources: GOC:dph, GOC:sdb_2009, GOC:tb Definition: The commitment of a cell to an endothelial cell fate and its capacity to differentiate into an endothelial cell. Relationships: is a type of epithelial cell fate commitment [GO:0072148]; is part of endothelial cell differentiation [GO:0045446] Subtypes: lymphatic endothelial cell fate commitment [GO:0060838], blood vessel endothelial cell fate commitment [GO:0060846], endocardial cell fate commitment [GO:0060957]